{
  "term_label": "Unknown cellular component",
  "gene_name": "Protein FAM182A",
  "term_id": "UNKNOWN:0003",
  "gene": "UniProtKB:Q5T1J6",
  "gene_symbol": "FAM182A"
}